{
  "gene": "UniProtKB:Q6IPR3",
  "term_id": "GO:0005737",
  "term_label": "cytoplasm",
  "gene_symbol": "TYW3",
  "gene_name": "tRNA wybutosine-synthesizing protein 3 homolog"
}